adventitious root development [GO:0048830] (biological process) Relationships: is a type of root development [GO:0048364] Definition: The process whose specific outcome is the progression of adventitious root over time, from its formation to the mature structure. Adventitious roots are post-embryonic roots that develop from the plant shoot. Sources: GOC:tb